{
  "gene": "UniProtKB:Q9H1V8",
  "term_id": "GO:0015816",
  "gene_name": "Sodium-dependent neutral amino acid transporter SLC6A17",
  "gene_symbol": "SLC6A17",
  "term_label": "glycine transport"
}